{
  "gene_symbol": "SGK1",
  "term_label": "neuron projection morphogenesis",
  "term_id": "GO:0048812",
  "gene": "UniProtKB:O00141",
  "gene_name": "Serine_threonine-protein kinase Sgk1"
}